2-isopropylmalate synthase activity [GO:0003852] (molecular function) Relationships: is a type of acyltransferase activity, acyl groups converted into alkyl on transfer [GO:0046912] Also known as: 3-carboxy-3-hydroxy-4-methylpentanoate 3-methyl-2-oxobutanoate-lyase (CoA-acetylating) activity, acetyl-CoA:3-methyl-2-oxobutanoate C-acetyltransferase (thioester-hydrolysing, carboxymethyl-forming), alpha-IPM synthetase activity, alpha-isopropylmalate synthase activity, alpha-isopropylmalate synthetase activity, alpha-isopropylmalic synthetase activity, isopropylmalate synthase activity, isopropylmalate synthetase activity Definition: Catalysis of the reaction: 3-methyl-2-oxobutanoate + acetyl-CoA + H2O = (2S)-2-isopropylmalate + CoA + H+. Sources: RHEA:21524